{
  "gene_symbol": "RSL24D1",
  "term_label": "ribosomal large subunit biogenesis",
  "gene_name": "Probable ribosome biogenesis protein RLP24",
  "term_id": "GO:0042273",
  "gene": "UniProtKB:Q9UHA3"
}